{
  "gene_symbol": "ARHGEF6",
  "term_id": "GO:0030027",
  "term_label": "lamellipodium",
  "gene_name": "Rho guanine nucleotide exchange factor 6",
  "gene": "UniProtKB:Q15052"
}